{
  "gene_symbol": "MCM10",
  "term_label": "single-stranded DNA binding",
  "gene_name": "Protein MCM10 homolog",
  "gene": "UniProtKB:Q7L590",
  "term_id": "GO:0003697"
}